{
  "gene": "UniProtKB:A2A3K4",
  "term_id": "GO:0005737",
  "gene_symbol": "PTPDC1",
  "term_label": "cytoplasm",
  "gene_name": "Protein tyrosine phosphatase domain-containing protein 1"
}